apical cytoplasm [GO:0090651] (cellular component) Definition: The region of the cytoplasm located at the apical side of the cell. Used in reference to animal polarized epithelial cells. References: PMID:17494872 Relationships: is a type of cellular anatomical structure [GO:0110165]; BFO_0000050 cytoplasm [GO:0005737]; is part of apical part of cell [GO:0045177]